{
  "gene": "UniProtKB:P28356",
  "gene_name": "Homeobox protein Hox-D9",
  "term_label": "embryonic skeletal system morphogenesis",
  "gene_symbol": "HOXD9",
  "term_id": "GO:0048704"
}